negative regulation of retrograde dense core granule transport [GO:1901955] (biological process) Definition: Any process that stops, prevents or reduces the frequency, rate or extent of retrograde dense core granule transport. Relationships: is a type of negative regulation of vesicle transport along microtubule [GO:1901609]; is a type of regulation of retrograde dense core granule transport [GO:1901954]; is a type of negative regulation of dense core granule transport [GO:1904810]; is a type of negative regulation of retrograde axon cargo transport [GO:2001018]; negatively regulates retrograde neuronal dense core vesicle transport [GO:1990049] Also known as: down regulation of retrograde dense core granule transport, down-regulation of retrograde dense core granule transport, downregulation of retrograde dense core granule transport, inhibition of retrograde dense core granule transport References: PMID:23358451 Sources: GOC:TermGenie, GOC:kmv